{
  "gene": "UniProtKB:Q9NPC2",
  "gene_name": "Potassium channel subfamily K member 9",
  "term_id": "GO:0015271",
  "gene_symbol": "KCNK9",
  "term_label": "outward rectifier potassium channel activity"
}